{
  "term_id": "GO:0016491",
  "term_label": "oxidoreductase activity",
  "gene_symbol": "SELENOF",
  "gene": "UniProtKB:O60613",
  "gene_name": "Selenoprotein F"
}